{
  "term_label": "ERBB2 signaling pathway",
  "gene": "UniProtKB:O75131",
  "term_id": "GO:0038128",
  "gene_symbol": "CPNE3",
  "gene_name": "Copine-3"
}